glucose-1-phosphate guanylyltransferase activity [GO:0047344] (molecular function) Definition: Catalysis of the reaction: alpha-D-glucose 1-phosphate + GTP = diphosphate + GDP-D-glucose. Also known as: GTP:glucose-1-phosphate guanylyltransferase activity, GDP glucose pyrophosphorylase activity, GDP-glucose diphosphorylase activity, GDP-glucose pyrophosphorylase activity, GTP:alpha-D-glucose-1-phosphate guanylyltransferase activity, guanosine diphosphoglucose pyrophosphorylase activity Sources: RHEA:10708 Relationships: is a type of guanylyltransferase activity [GO:0070568]